{
  "gene": "UniProtKB:P56270",
  "term_id": "UNKNOWN:0003",
  "term_label": "Unknown cellular component",
  "gene_name": "Myc-associated zinc finger protein",
  "gene_symbol": "MAZ"
}